{
  "gene_symbol": "IGF2BP2",
  "gene_name": "Insulin-like growth factor 2 mRNA-binding protein 2",
  "term_label": "mRNA 3'-UTR binding",
  "gene": "UniProtKB:Q9Y6M1",
  "term_id": "GO:0003730"
}